{
  "term_label": "unsaturated fatty acid biosynthetic process",
  "gene_name": "Stearoyl-CoA desaturase",
  "term_id": "GO:0006636",
  "gene": "UniProtKB:O00767",
  "gene_symbol": "SCD"
}